{
  "term_label": "negative regulation of apoptotic process",
  "gene_symbol": "PTMA",
  "gene_name": "Prothymosin alpha",
  "gene": "UniProtKB:P06454",
  "term_id": "GO:0043066"
}